diadenosine triphosphate biosynthetic process [GO:0015963] (biological process) Definition: The chemical reactions and pathways resulting in the formation of diadenosine triphosphate, a derivative of the nucleoside adenosine with three phosphate groups attached. Also known as: diadenosine triphosphate anabolism, diadenosine triphosphate biosynthesis, diadenosine triphosphate formation, diadenosine triphosphate synthesis Relationships: is a type of diadenosine polyphosphate biosynthetic process [GO:0015960] Sources: GOC:ai